{
  "gene_name": "Kinetochore scaffold 1",
  "term_id": "UNKNOWN:0001",
  "term_label": "Unknown molecular function",
  "gene_symbol": "KNL1",
  "gene": "UniProtKB:Q8NG31"
}